{
  "term_label": "mitochondrial electron transport, NADH to ubiquinone",
  "gene": "UniProtKB:O95182",
  "gene_symbol": "NDUFA7",
  "gene_name": "NADH dehydrogenase [ubiquinone] 1 alpha subcomplex subunit 7",
  "term_id": "GO:0006120"
}